myosin I tail binding [GO:0032032] (molecular function) Relationships: is a type of myosin tail binding [GO:0032029]; is a type of myosin I heavy chain binding [GO:0032037] Sources: GOC:mah Definition: Binding to the tail region of a myosin I heavy chain.